{
  "term_label": "ubiquitin conjugating enzyme activity",
  "gene_symbol": "UBE2C",
  "gene": "UniProtKB:O00762",
  "term_id": "GO:0061631",
  "gene_name": "Ubiquitin-conjugating enzyme E2 C"
}